glutathione-homocystine transhydrogenase activity [GO:0047139] (molecular function) Relationships: is a type of GO:0016671 Also known as: glutathione:homocystine oxidoreductase activity Sources: EC:1.8.4.1, MetaCyc:1.8.4.1-RXN Definition: Catalysis of the reaction: homocystine + 2 reduced glutathione = oxidized glutathione + 2 homocysteine.